{
  "gene_symbol": "IGFBP1",
  "term_id": "GO:0031994",
  "gene_name": "Insulin-like growth factor-binding protein 1",
  "term_label": "insulin-like growth factor I binding",
  "gene": "UniProtKB:P08833"
}